{
  "term_label": "Unknown biological process",
  "gene": "UniProtKB:Q0PNE2",
  "gene_name": "Elongator complex protein 6",
  "gene_symbol": "ELP6",
  "term_id": "UNKNOWN:0002"
}